channel complex [GO:0170013] (cellular component) Relationships: is a type of membrane protein complex [GO:0098796] Definition: A protein complex that spans a membrane and forms a water-filled channel across the phospholipid bilayer allowing selective ion transport down its electrochemical gradient. References: PMID:10839820